{
  "gene_symbol": "RBMXL2",
  "gene_name": "RNA-binding motif protein, X-linked-like-2",
  "term_label": "mRNA binding",
  "gene": "UniProtKB:O75526",
  "term_id": "GO:0003729"
}